{
  "gene": "UniProtKB:Q96G30",
  "term_id": "GO:0031782",
  "term_label": "type 4 melanocortin receptor binding",
  "gene_symbol": "MRAP2",
  "gene_name": "Melanocortin-2 receptor accessory protein 2"
}